basophil activation [GO:0045575] (biological process) Subtypes: basophil activation involved in immune response [GO:0002276] Relationships: is a type of GO:0036230 Definition: The change in morphology and behavior of a basophil resulting from exposure to a cytokine, chemokine, soluble factor, or to (at least in mammals) an antigen which the basophil has specifically bound via IgE bound to Fc-epsilonRI receptors. Sources: GOC:mgi_curators, ISBN:0781735149